serotonin uptake [GO:0051610] (biological process) Definition: The directed movement of serotonin into a cell, typically presynaptic neurons or glial cells. Serotonin (5-hydroxytryptamine) is a monoamine neurotransmitter occurring in the peripheral and central nervous systems. Sources: GOC:ai Also known as: 5-HT uptake, 5-hydroxytryptamine uptake, 5HT uptake, serotonin import Regulation: regulated by GO:0051611; negatively regulated by GO:0051612; positively regulated by positive regulation of serotonin uptake [GO:0051613] Relationships: is a type of serotonin transport [GO:0006837]; is a type of GO:0098810